regulation of arachidonate secretion [GO:0090237] (biological process) Relationships: is a type of GO:0032303; regulates arachidonate secretion [GO:0050482] Definition: Any process that modulates the rate, frequency, or extent of arachidonic acid secretion, the controlled release of arachidonic acid from a cell or a tissue. Subtypes: GO:0090238, GO:1900139 Sources: GOC:dph, GOC:tb Also known as: regulation of arachidonic acid secretion